{
  "gene": "UniProtKB:Q12816",
  "gene_symbol": "TRO",
  "gene_name": "Trophinin",
  "term_label": "nucleus",
  "term_id": "GO:0005634"
}